formation of tubovesicular network for nutrient acquisition [GO:0085019] (biological process) Sources: GOC:pamgo_curators Also known as: formation of a symbiont- induced tubovesicular network for nutrient acquisition from host, formation by symbiont of a tubovesicular network for nutrient acquisition from host Relationships: is a type of formation of specialized structure for nutrient acquisition [GO:0052093] Definition: The assembly of a symbiont-induced complex organelle that comprises of multiple protein and lipid domains for the purpose of obtaining nutrients from its host organism. The host is defined as the larger of the organisms involved in a symbiotic interaction.